{
  "gene_symbol": "EHD2",
  "term_label": "recycling endosome membrane",
  "gene_name": "EH domain-containing protein 2",
  "term_id": "GO:0055038",
  "gene": "UniProtKB:Q9NZN4"
}